{
  "gene_name": "Actin-binding LIM protein 2",
  "term_id": "GO:0051015",
  "gene_symbol": "ABLIM2",
  "gene": "UniProtKB:Q6H8Q1",
  "term_label": "actin filament binding"
}